Notch binding [GO:0005112] (molecular function) Relationships: is a type of GO:0005102 Definition: Binding to a Notch (N) protein, a surface receptor. Also known as: N binding, Notch receptor binding, N ligand, Notch ligand Sources: GOC:ceb